{
  "term_label": "Unknown molecular function",
  "gene_symbol": "ANXA2R",
  "gene_name": "Annexin-2 receptor",
  "gene": "UniProtKB:Q3ZCQ2",
  "term_id": "UNKNOWN:0001"
}